{
  "term_id": "GO:0048010",
  "gene": "UniProtKB:P15692",
  "term_label": "vascular endothelial growth factor receptor signaling pathway",
  "gene_symbol": "VEGFA",
  "gene_name": "Vascular endothelial growth factor A, long form"
}